{
  "gene_symbol": "DEFB115",
  "gene_name": "Beta-defensin 115",
  "term_label": "membrane destabilizing activity",
  "gene": "UniProtKB:Q30KQ5",
  "term_id": "GO:0140912"
}